citrate transmembrane transporter activity [GO:0015137] (molecular function) Relationships: is a type of tricarboxylic acid transmembrane transporter activity [GO:0015142]; is part of citrate transport [GO:0015746] Also known as: tricarboxylate transport protein Definition: Enables the transfer of citrate, 2-hydroxy-1,2,3-propanetricarboxylate, from one side of a membrane to the other. Sources: GOC:ai Subtypes: citrate secondary active transmembrane transporter activity [GO:0071913]